{
  "gene_name": "Zinc finger MYND domain-containing protein 10",
  "term_label": "outer dynein arm assembly",
  "gene": "UniProtKB:O75800",
  "gene_symbol": "ZMYND10",
  "term_id": "GO:0036158"
}